positive regulation of fatty acid beta-oxidation [GO:0032000] (biological process) Sources: GOC:mah Definition: Any process that activates or increases the frequency, rate or extent of fatty acid beta-oxidation. Relationships: is a type of regulation of fatty acid beta-oxidation [GO:0031998]; is a type of positive regulation of fatty acid oxidation [GO:0046321]; is a type of positive regulation of lipid catabolic process [GO:0050996]; positively regulates fatty acid beta-oxidation [GO:0006635] Also known as: up regulation of fatty acid beta-oxidation, up-regulation of fatty acid beta-oxidation, upregulation of fatty acid beta-oxidation, activation of fatty acid beta-oxidation, stimulation of fatty acid beta-oxidation Subtypes: GO:1904122, positive regulation of fatty acid beta-oxidation by serotonin receptor signaling pathway [GO:1904123], GO:1904737